1,6-dihydroxycyclohexa-2,4-diene-1-carboxylate dehydrogenase activity [GO:0047116] (molecular function) Sources: EC:1.3.1.25, MetaCyc:1.3.1.25-RXN Relationships: is a type of GO:0016628 Definition: Catalysis of the reaction: NAD+ + 1,6-dihydroxycyclohexa-2,4-diene-1-carboxylate = NADH + CO2 + catechol. Also known as: (1R,6R)-1,6-dihydroxycyclohexa-2,4-diene-1-carboxylate:NAD+ oxidoreductase (decarboxylating), 2-hydro-1,2-dihydroxybenzoate dehydrogenase activity, 3,5-cyclohexadiene-1,2-diol-1-carboxylate dehydrogenase activity, 3,5-cyclohexadiene-1,2-diol-1-carboxylic acid dehydrogenase activity, DHB dehydrogenase activity, DHBDH activity, cis-1,2-dihydroxycyclohexa-3,5-diene-1-carboxylate:NAD(+) oxidoreductase activity, cis-1,2-dihydroxycyclohexa-3,5-diene-1-carboxylate:NAD+ oxidoreductase activity, dihydrodihydroxybenzoate dehydrogenase activity